mitochondrial respiratory chain complex IV pre-assembly complex [GO:0062011] (cellular component) Definition: A protein complex that contributes to and regulates mitochondrial respiratory chain complex IV (COX) formation. It acts by regulating mitochondrial COX1 translation and by promoting the assembly of COX components. References: PMID:21068384 Sources: GOC:lnp Also known as: COX pre-assemply complex, COX1 preassemply complex Relationships: is a type of inner mitochondrial membrane protein complex [GO:0098800]; is a type of protein folding chaperone complex [GO:0101031]